negative regulation of lymphangiogenesis [GO:1901491] (BP) Definition: Any process that stops, prevents or reduces the frequency, rate or extent of lymphangiogenesis. References: PMID:20133819 Sources: GOC:TermGenie, GOC:dph Also known as: down regulation of lymph vessel formation, down regulation of lymphangiogenesis, down-regulation of lymph vessel formation, down-regulation of lymphangiogenesis, downregulation of lymph vessel formation, downregulation of lymphangiogenesis, negative regulation of lymph vessel formation, inhibition of lymph vessel formation, inhibition of lymphangiogenesis Relationships: is a type of GO:0051093; is a type of regulation of lymphangiogenesis [GO:1901490]; RO_0002212 lymphangiogenesis [GO:0001946]